{
  "term_id": "GO:0000977",
  "gene_symbol": "ZNF669",
  "gene_name": "Zinc finger protein 669",
  "term_label": "RNA polymerase II transcription regulatory region sequence-specific DNA binding",
  "gene": "UniProtKB:Q96BR6"
}